chemokine (C-C motif) ligand 5 binding [GO:0071791] (molecular function) Sources: GOC:add, GOC:amm Definition: Binding to chemokine (C-C motif) ligand 5. Relationships: is a type of C-C chemokine binding [GO:0019957] Also known as: CCL5 binding, RANTES binding, Regulated upon Activation, Normal T-cell Expressed, and Secreted binding